{
  "term_id": "UNKNOWN:0001",
  "gene_name": "Golgin subfamily A member 8B",
  "term_label": "Unknown molecular function",
  "gene": "UniProtKB:A8MQT2",
  "gene_symbol": "GOLGA8B"
}